response to antibiotic [GO:0046677] (biological process) Also known as: antibiotic susceptibility/resistance Definition: Any process that results in a change in state or activity of a cell or an organism (in terms of movement, secretion, enzyme production, gene expression, etc.) as a result of an antibiotic stimulus. An antibiotic is a chemical substance produced by a microorganism which has the capacity to inhibit the growth of or to kill other microorganisms. Subtypes: GO:0031001, response to trichostatin A [GO:0035983], response to bacteriocin [GO:0046678], response to streptomycin [GO:0046679], GO:0060992, GO:0061479, cellular response to antibiotic [GO:0071236], GO:0072716 Relationships: is a type of response to chemical [GO:0042221] Sources: GOC:ai, GOC:ef